{
  "gene": "UniProtKB:Q9BZF9",
  "term_id": "GO:1901223",
  "gene_name": "Uveal autoantigen with coiled-coil domains and ankyrin repeats",
  "gene_symbol": "UACA",
  "term_label": "negative regulation of non-canonical NF-kappaB signal transduction"
}